{
  "gene": "UniProtKB:P79483",
  "gene_symbol": "HLA-DRB3",
  "gene_name": "HLA class II histocompatibility antigen, DR beta 3 chain",
  "term_id": "GO:0042605",
  "term_label": "peptide antigen binding"
}